GARP complex [GO:0000938] (cellular component) Relationships: is_a vesicle tethering complex [GO:0099023]; is part of GO:0005794; is part of GO:0031410 Also known as: Golgi associated retrograde protein complex, VFT tethering complex, Vps fifty three tethering complex References: PMID:10637310, PMID:12077354, PMID:12446664 Sources: GOC:clt, GOC:rn Definition: A quatrefoil tethering complex required for retrograde traffic from the early endosome back to the late Golgi and biogenesis of cytoplasmic vesicles.